{
  "gene": "UniProtKB:Q9HCE0",
  "gene_symbol": "EPG5",
  "term_label": "Unknown molecular function",
  "gene_name": "Ectopic P granules protein 5 homolog",
  "term_id": "UNKNOWN:0001"
}